{
  "term_id": "GO:0006241",
  "gene": "UniProtKB:P17812",
  "gene_name": "CTP synthase 1",
  "gene_symbol": "CTPS1",
  "term_label": "CTP biosynthetic process"
}